MAP kinase tyrosine phosphatase activity [GO:0033550] (molecular function) Definition: Catalysis of the reaction: MAP kinase tyrosine phosphate + H2O = MAP kinase tyrosine + phosphate. Also known as: tyrosine-specific MAP kinase phosphatase activity Relationships: is a type of protein tyrosine phosphatase activity [GO:0004725]; is_a GO:0033549 Sources: GOC:mah